3-(2,3-dihydroxyphenyl)propanoate biosynthetic process [GO:1901792] (biological process) Definition: The chemical reactions and pathways resulting in the formation of 3-(2,3-dihydroxyphenyl)propanoate. Also known as: 3-(2,3-dihydroxyphenyl)propanoate anabolism, 3-(2,3-dihydroxyphenyl)propanoate biosynthesis, 3-(2,3-dihydroxyphenyl)propanoate formation, 3-(2,3-dihydroxyphenyl)propanoate synthesis Relationships: is a type of catechol-containing compound biosynthetic process [GO:0009713]; is a type of monocarboxylic acid biosynthetic process [GO:0072330] Sources: GOC:TermGenie, GOC:yaf